{
  "term_label": "RNA polymerase II cis-regulatory region sequence-specific DNA binding",
  "gene_symbol": "KRBOX4",
  "gene": "UniProtKB:Q5JUW0",
  "term_id": "GO:0000978",
  "gene_name": "KRAB domain-containing protein 4"
}